{
  "term_id": "GO:0030314",
  "gene": "UniProtKB:Q9HDC5",
  "gene_name": "Junctophilin-1",
  "gene_symbol": "JPH1",
  "term_label": "junctional membrane complex"
}